actomyosin contractile ring assembly actin filament bundle convergence [GO:0071520] (biological process) Also known as: actin filament bundle convergence involved in cytokinetic actomyosin contractile ring assembly, actin filament bundle convergence involved in actomyosin contractile ring formation Relationships: is a type of GO:0090426; is a type of actomyosin contractile ring assembly actin filament organization [GO:2000689] References: PMID:19713940 Sources: GOC:mah Definition: A process of actin filament bundle distribution that occurs in the context of assembling an actomyosin contractile ring during cytokinesis, and that results in the compaction of actin filaments into a tight ring.